{
  "gene": "UniProtKB:Q9BTP7",
  "term_label": "chromatin binding",
  "term_id": "GO:0003682",
  "gene_symbol": "FAAP24",
  "gene_name": "Fanconi anemia core complex-associated protein 24"
}